{
  "term_label": "T cell differentiation",
  "gene_name": "Tyrosine-protein kinase Lck",
  "gene_symbol": "LCK",
  "gene": "UniProtKB:P06239",
  "term_id": "GO:0030217"
}